{
  "gene_symbol": "RNF183",
  "gene_name": "E3 ubiquitin-protein ligase RNF183",
  "term_label": "endoplasmic reticulum membrane",
  "gene": "UniProtKB:Q96D59",
  "term_id": "GO:0005789"
}